{
  "term_id": "GO:0006955",
  "term_label": "immune response",
  "gene_symbol": "CLEC4M",
  "gene": "UniProtKB:Q9H2X3",
  "gene_name": "C-type lectin domain family 4 member M"
}